{
  "term_id": "GO:0072686",
  "gene_name": "Echinoderm microtubule-associated protein-like 1",
  "gene": "UniProtKB:O00423",
  "term_label": "mitotic spindle",
  "gene_symbol": "EML1"
}